{
  "gene": "UniProtKB:O60315",
  "gene_symbol": "ZEB2",
  "term_label": "regulation of transcription by RNA polymerase II",
  "term_id": "GO:0006357",
  "gene_name": "Zinc finger E-box-binding homeobox 2"
}